acryloyl-CoA reductase (NADH) activity [GO:0043958] (molecular function) References: PMID:12603323 Sources: GOC:jl Note: Note that this function is part of the process of L-alanine fermentation to propionate. Also known as: acryloyl-CoA reductase activity, acryloyl-coenzyme A reductase activity, propionyl-CoA dehydrogenase, acrylyl-CoA reductase (NADH) Definition: Catalysis of the reaction: propanoyl-CoA + NAD+ = acryloyl-CoA + H+ + NADH. Relationships: is a type of oxidoreductase activity, acting on the CH-CH group of donors, NAD or NADP as acceptor [GO:0016628]